{
  "gene_name": "Transmembrane protein 33",
  "term_id": "GO:0005783",
  "gene": "UniProtKB:P57088",
  "gene_symbol": "TMEM33",
  "term_label": "endoplasmic reticulum"
}